{
  "gene_name": "Proto-oncogene Wnt-1",
  "gene": "UniProtKB:P04628",
  "term_id": "GO:0030182",
  "term_label": "neuron differentiation",
  "gene_symbol": "WNT1"
}